{
  "gene_name": "Myosin light chain kinase family member 4",
  "term_label": "myosin light chain kinase activity",
  "gene_symbol": "MYLK4",
  "term_id": "GO:0004687",
  "gene": "UniProtKB:Q86YV6"
}